mating [GO:0007618] (biological process) Relationships: is a type of multi-organism reproductive process [GO:0044703]; is part of sexual reproduction [GO:0019953] Sources: GOC:jl, ISBN:0387520546 Definition: The pairwise union of individuals for the purpose of sexual reproduction, ultimately resulting in the formation of zygotes.